{
  "gene_name": "Pro-neuregulin-2, membrane-bound isoform",
  "gene_symbol": "NRG2",
  "term_label": "ERBB4 signaling pathway",
  "gene": "UniProtKB:O14511",
  "term_id": "GO:0038130"
}